{
  "gene_name": "Eomesodermin homolog",
  "gene_symbol": "EOMES",
  "gene": "UniProtKB:O95936",
  "term_label": "regulation of transcription by RNA polymerase II",
  "term_id": "GO:0006357"
}